{
  "term_id": "GO:0015232",
  "gene_name": "Heme transporter FLVCR1",
  "gene": "UniProtKB:Q9Y5Y0",
  "gene_symbol": "FLVCR1",
  "term_label": "heme transmembrane transporter activity"
}